thromboxane transport [GO:0071717] (biological process) Subtypes: sodium-independent thromboxane transport [GO:0071721] Definition: The directed movement of thromboxanes into, out of or within a cell, or between cells, by means of some agent such as a transporter or pore. A thromboxane is any of a class of oxygenated oxane derivatives, originally derived from prostaglandin precursors in platelets, that stimulate aggregation of platelets and constriction of blood vessels. Sources: GOC:mah Relationships: is a type of fatty acid transport [GO:0015908]; is a type of icosanoid transport [GO:0071715]